{
  "gene_symbol": "RANBP1",
  "gene_name": "Ran-specific GTPase-activating protein",
  "term_label": "Unknown molecular function",
  "gene": "UniProtKB:P43487",
  "term_id": "UNKNOWN:0001"
}